epithelial cell proliferation involved in lung bud dilation [GO:0060505] (biological process) Sources: GOC:dph Relationships: is_a epithelial cell proliferation involved in lung morphogenesis [GO:0060502]; is part of bud dilation involved in lung branching [GO:0060503] Definition: The multiplication or reproduction of epithelial cells that contribute to the radial growth of a lung bud. Regulation: positively regulated by positive regulation of epithelial cell proliferation involved in lung bud dilation [GO:0060504]